{
  "gene_symbol": "FRAS1",
  "term_id": "GO:0031012",
  "gene": "UniProtKB:Q86XX4",
  "term_label": "extracellular matrix",
  "gene_name": "Extracellular matrix organizing protein FRAS1"
}